{
  "term_id": "UNKNOWN:0003",
  "gene_name": "HEAT repeat-containing protein 4",
  "term_label": "Unknown cellular component",
  "gene": "UniProtKB:Q86WZ0",
  "gene_symbol": "HEATR4"
}